{
  "gene_name": "Peroxisomal membrane protein PEX16",
  "term_label": "peroxisomal membrane",
  "gene": "UniProtKB:Q9Y5Y5",
  "term_id": "GO:0005778",
  "gene_symbol": "PEX16"
}